{
  "gene_name": "Condensin-2 complex subunit D3",
  "term_label": "condensin complex",
  "term_id": "GO:0000796",
  "gene_symbol": "NCAPD3",
  "gene": "UniProtKB:P42695"
}